{
  "term_id": "GO:0019814",
  "gene_symbol": "TRAV8-2",
  "gene": "UniProtKB:A0A0B4J237",
  "gene_name": "T cell receptor alpha variable 8-2",
  "term_label": "immunoglobulin complex"
}